{
  "term_id": "GO:0006302",
  "gene_symbol": "MTA1",
  "term_label": "double-strand break repair",
  "gene": "UniProtKB:Q13330",
  "gene_name": "Metastasis-associated protein MTA1"
}